{
  "gene": "UniProtKB:O43193",
  "term_id": "GO:0008528",
  "gene_symbol": "MLNR",
  "gene_name": "Motilin receptor",
  "term_label": "G protein-coupled peptide receptor activity"
}